mammary gland formation [GO:0060592] (BP) Subtypes: mammary gland specification [GO:0060594] Definition: The process pertaining to the initial formation of the mammary gland from unspecified parts. The process begins with formation of the mammary line and ends when the solid mammary bud invades the primary mammary mesenchyme. Relationships: is_a anatomical structure formation involved in morphogenesis [GO:0048646]; is part of GO:0060443 References: PMID:16168142, PMID:17120154 Sources: GOC:dph Also known as: mammary line formation, mammary placode formation, mammary bud formation, mammary sprout formation